detection of mechanical stimulus involved in sensory perception of wind [GO:0071066] (biological process) Relationships: is a type of nervous system process [GO:0050877]; is a type of GO:0050974; is part of sensory perception of wind [GO:0071063] Also known as: detection of mechanical stimulus involved in sensory perception of air flow, detection of wind, perception of wind, detection of mechanical stimulus, perception of wind, sensory detection of mechanical stimulus, perception of wind, sensory transduction of mechanical stimulus, sensory detection of mechanical stimulus during perception of wind, sensory transduction of mechanical stimulus during perception of wind, sensory transduction of wind References: PMID:19279637 Sources: GOC:dos, GOC:mah Definition: The series of events involved in the perception of wind in which a mechanical stimulus is received and converted into a molecular signal.